{
  "term_label": "cytoplasm",
  "gene_name": "Mth938 domain-containing protein",
  "term_id": "GO:0005737",
  "gene_symbol": "AAMDC",
  "gene": "UniProtKB:Q9H7C9"
}